{
  "gene": "UniProtKB:Q14032",
  "gene_name": "Bile acid-CoA:amino acid N-acyltransferase",
  "term_id": "GO:0006631",
  "term_label": "fatty acid metabolic process",
  "gene_symbol": "BAAT"
}